neuronal action potential back-propagation [GO:0098873] (biological process) Definition: Propagation of an action potential in a neuron, from its site of initiation (typically the axon hillock) towards the soma. Sources: GOC:dos Relationships: is a type of GO:0098870